{
  "term_id": "UNKNOWN:0001",
  "gene_name": "Putative uncharacterized protein SHANK2-AS3",
  "gene": "UniProtKB:Q9BTD1",
  "gene_symbol": "SHANK2-AS3",
  "term_label": "Unknown molecular function"
}